regulation of microtubule-based movement [GO:0060632] (BP) Sources: GOC:dph, GOC:tb Subtypes: regulation of cilium movement [GO:0003352], regulation of plus-end directed microtubule sliding [GO:0062169], regulation of organelle transport along microtubule [GO:1902513], GO:1905126, regulation of intraciliary anterograde transport [GO:1905796], regulation of intraciliary retrograde transport [GO:1905799], GO:2001017 Definition: Any process that modulates the rate, frequency, or extent of microtubule-based movement, the movement of organelles, other microtubules and other particles along microtubules, mediated by motor proteins. Relationships: is a type of GO:0032886; regulates microtubule-based movement [GO:0007018]